{
  "gene_symbol": "ZNF235",
  "gene": "UniProtKB:Q14590",
  "gene_name": "Zinc finger protein 235",
  "term_id": "UNKNOWN:0002",
  "term_label": "Unknown biological process"
}